dendrite membrane [GO:0032590] (cellular component) Relationships: is_a neuron projection membrane [GO:0032589]; is part of GO:0030425 Definition: The portion of the plasma membrane surrounding a dendrite. Sources: GOC:mah